{
  "term_id": "UNKNOWN:0001",
  "gene_symbol": "ROM1",
  "term_label": "Unknown molecular function",
  "gene_name": "Rod outer segment membrane protein 1",
  "gene": "UniProtKB:Q03395"
}